{
  "gene_symbol": "FAM167A-AS1",
  "gene": "UniProtKB:Q96KT0",
  "gene_name": "Uncharacterized protein FAM167A-AS1",
  "term_id": "UNKNOWN:0002",
  "term_label": "Unknown biological process"
}